{
  "gene_symbol": "ZNF295-AS1",
  "gene": "UniProtKB:Q8N0V1",
  "term_label": "Unknown biological process",
  "term_id": "UNKNOWN:0002",
  "gene_name": "Putative uncharacterized protein ZNF295-AS1"
}